{
  "term_id": "GO:0038191",
  "gene": "UniProtKB:Q9NPR2",
  "gene_symbol": "SEMA4B",
  "term_label": "neuropilin binding",
  "gene_name": "Semaphorin-4B"
}